{
  "gene": "UniProtKB:A6NDR6",
  "term_label": "RNA polymerase II cis-regulatory region sequence-specific DNA binding",
  "gene_name": "Putative homeobox protein Meis3-like 1",
  "gene_symbol": "MEIS3P1",
  "term_id": "GO:0000978"
}